{
  "term_id": "UNKNOWN:0003",
  "gene_symbol": "CRYGS",
  "term_label": "Unknown cellular component",
  "gene_name": "Gamma-crystallin S",
  "gene": "UniProtKB:P22914"
}